{
  "term_label": "protein polyubiquitination",
  "gene_name": "WD repeat and SOCS box-containing protein 2",
  "term_id": "GO:0000209",
  "gene": "UniProtKB:Q9NYS7",
  "gene_symbol": "WSB2"
}